{
  "gene_symbol": "POLR3C",
  "gene_name": "DNA-directed RNA polymerase III subunit RPC3",
  "term_id": "UNKNOWN:0002",
  "gene": "UniProtKB:Q9BUI4",
  "term_label": "Unknown biological process"
}